{
  "gene_symbol": "NUDT10",
  "gene_name": "Diphosphoinositol polyphosphate phosphohydrolase 3-alpha",
  "term_id": "GO:0005634",
  "gene": "UniProtKB:Q8NFP7",
  "term_label": "nucleus"
}